{
  "gene": "UniProtKB:Q93079",
  "gene_symbol": "H2BC9",
  "term_label": "structural constituent of chromatin",
  "term_id": "GO:0030527",
  "gene_name": "Histone H2B type 1-H"
}